{
  "gene_name": "Testis-expressed protein 19",
  "gene": "UniProtKB:Q8NA77",
  "term_label": "cytoplasm",
  "gene_symbol": "TEX19",
  "term_id": "GO:0005737"
}